shikimate 3-dehydrogenase (NADP+) activity [GO:0004764] (molecular function) Relationships: is a type of oxidoreductase activity, acting on the CH-OH group of donors, NAD or NADP as acceptor [GO:0016616] Also known as: DHS reductase activity, dehydroshikimic reductase activity, shikimate oxidoreductase activity, shikimate:NADP(+) oxidoreductase activity, 5-dehydroshikimate reductase activity, 5-dehydroshikimic reductase activity, shikimate:NADP(+) 5-oxidoreductase activity Sources: EC:1.1.1.25 Definition: Catalysis of the reaction: shikimate + NADP+ = 3-dehydroshikimate + NADPH + H+.